male-specific antibacterial humoral response [GO:0006962] (biological process) Definition: An immune response against bacteria, specific to males and mediated through a body fluid. Sources: GOC:go_curators Relationships: is a type of antibacterial humoral response [GO:0019731]; is a type of male-specific defense response to bacterium [GO:0050831]